protocadherin-alpha-v4-protocadherin-gamma-b4 complex [GO:0071187] (cellular component) References: PMID:15347688 Relationships: is a type of protocadherin-alpha-protocadherin-gamma complex [GO:0071183] Also known as: Pcdhga1-Pcdhgb4 complex Definition: A protein complex that contains the cell adhesion molecules protocadherin-alpha-v4 and protocadherin-gamma-b4, and is involved in the regulation of protein localization to the plasma membrane.